{
  "gene_symbol": "JSRP1",
  "term_label": "sarcoplasmic reticulum",
  "term_id": "GO:0016529",
  "gene_name": "Junctional sarcoplasmic reticulum protein 1",
  "gene": "UniProtKB:Q96MG2"
}